{
  "term_id": "GO:0007507",
  "term_label": "heart development",
  "gene_symbol": "SMYD2",
  "gene": "UniProtKB:Q9NRG4",
  "gene_name": "N-lysine methyltransferase SMYD2"
}